{
  "gene_name": "Phospholipase A and acyltransferase 5",
  "term_id": "GO:0005737",
  "gene_symbol": "PLAAT5",
  "gene": "UniProtKB:Q96KN8",
  "term_label": "cytoplasm"
}